{
  "gene": "UniProtKB:P48552",
  "term_label": "nuclear retinoid X receptor binding",
  "gene_name": "Nuclear receptor-interacting protein 1",
  "term_id": "GO:0046965",
  "gene_symbol": "NRIP1"
}